{
  "gene_symbol": "CD180",
  "term_label": "cellular response to lipopolysaccharide",
  "gene_name": "CD180 antigen",
  "gene": "UniProtKB:Q99467",
  "term_id": "GO:0071222"
}